{
  "gene": "UniProtKB:Q13485",
  "gene_symbol": "SMAD4",
  "term_id": "GO:0007179",
  "term_label": "transforming growth factor beta receptor signaling pathway",
  "gene_name": "Mothers against decapentaplegic homolog 4"
}